glyoxysome organization [GO:0010111] (biological process) Definition: A process that is carried out at the cellular level which results in the assembly, arrangement of constituent parts, or disassembly of the glyoxysome. A glyoxysome is a microbody that contains the enzymes of the glyoxylate pathway. Relationships: is a type of GO:0007031; is a type of plastid organization [GO:0009657] Also known as: glyoxysome organisation, glyoxysome organization and biogenesis Sources: GOC:tb